{
  "gene_symbol": "PIK3C2G",
  "gene_name": "Phosphatidylinositol 3-kinase C2 domain-containing subunit gamma",
  "gene": "UniProtKB:O75747",
  "term_id": "GO:0043491",
  "term_label": "phosphatidylinositol 3-kinase/protein kinase B signal transduction"
}